{
  "term_id": "GO:0000165",
  "gene_symbol": "TAOK3",
  "gene": "UniProtKB:Q9H2K8",
  "term_label": "MAPK cascade",
  "gene_name": "Serine_threonine-protein kinase TAO3"
}